{
  "term_label": "DNA methylation-dependent constitutive heterochromatin formation",
  "gene_symbol": "MBD3L2",
  "term_id": "GO:0006346",
  "gene_name": "Methyl-CpG-binding domain protein 3-like 2",
  "gene": "UniProtKB:Q8NHZ7"
}